snoRNA localization [GO:0048254] (biological process) Definition: Any process in which small nucleolar RNA is transported to, or maintained in, a specific location. Sources: ISBN:0716731363 Relationships: is a type of GO:0006403 Also known as: establishment and maintenance of snoRNA localization, small nucleolar RNA localization, snoRNA localisation